positive regulation of cardiac epithelial to mesenchymal transition [GO:0062043] (biological process) Relationships: is a type of positive regulation of epithelial to mesenchymal transition [GO:0010718]; is a type of regulation of cardiac epithelial to mesenchymal transition [GO:0062042]; positively regulates cardiac epithelial to mesenchymal transition [GO:0060317] Subtypes: positive regulation of endocardial cushion to mesenchymal transition [GO:0140051], positive regulation of epithelial to mesenchymal transition involved in endocardial cushion formation [GO:1905007] References: PMID:20951801 Sources: GOC:BHF, GOC:rph Definition: Any process that starts or increases the rate, frequency or extent of cardiac epithelial to mesenchymal transition, a transition where a cardiac epithelial cell loses apical/basolateral polarity, severs intercellular adhesive junctions, degrades basement membrane components and becomes a migratory mesenchymal cell.